{
  "gene_name": "Integrator complex subunit 6",
  "term_id": "GO:0034472",
  "term_label": "snRNA 3'-end processing",
  "gene": "UniProtKB:Q9UL03",
  "gene_symbol": "INTS6"
}